{
  "gene_name": "Mothers against decapentaplegic homolog 9",
  "term_label": "regulation of transcription by RNA polymerase II",
  "gene_symbol": "SMAD9",
  "term_id": "GO:0006357",
  "gene": "UniProtKB:O15198"
}